{
  "term_label": "ephrin receptor signaling pathway",
  "gene": "UniProtKB:P54756",
  "gene_name": "Ephrin type-A receptor 5",
  "term_id": "GO:0048013",
  "gene_symbol": "EPHA5"
}